pre-tubular aggregate formation [GO:0072035] (biological process) Sources: GOC:mtg_kidney_jan10 Regulation: RO_0002211 by regulation of pre-tubular aggregate formation by cell-cell signaling [GO:0072043] Relationships: is a type of cell-cell adhesion [GO:0098609]; is part of GO:0072033 Also known as: mesenchymal cell condensation involved in renal vesicle formation, nephron epithelium formation Definition: The cell adhesion process in which mesenchyme cells adhere to one another in the initial stages of the formation of the pre-tubular aggregate, the earliest recognizable structure of the kidney.